{
  "gene": "UniProtKB:Q9NVH0",
  "term_id": "GO:0005634",
  "term_label": "nucleus",
  "gene_name": "Exonuclease 3'-5' domain-containing protein 2",
  "gene_symbol": "EXD2"
}